{
  "term_label": "recycling endosome membrane",
  "gene_name": "Secretory carrier-associated membrane protein 4",
  "gene": "UniProtKB:Q969E2",
  "gene_symbol": "SCAMP4",
  "term_id": "GO:0055038"
}